{
  "gene_symbol": "BTNL9",
  "gene": "UniProtKB:Q6UXG8",
  "term_id": "GO:0001817",
  "gene_name": "Butyrophilin-like protein 9",
  "term_label": "regulation of cytokine production"
}